{
  "term_id": "GO:0000209",
  "gene_name": "Ubiquitin conjugation factor E4 B",
  "gene_symbol": "UBE4B",
  "term_label": "protein polyubiquitination",
  "gene": "UniProtKB:O95155"
}